glycerol-1-phosphate dehydrogenase [NAD(P)+] activity [GO:0050492] (molecular function) Subtypes: GO:0106357, glycerol-1-phosphate dehydrogenase (NADP+) activity [GO:0106358] Also known as: sn-glycerol-1-phosphate:NAD(P)+ 2-oxidoreductase activity Sources: EC:1.1.1.261 Definition: Catalysis of the reaction: NAD(P)+ + sn-glycerol-1-phosphate = NAD(P)H + H+ + dihydroxy-acetone-phosphate. Relationships: is a type of oxidoreductase activity, acting on the CH-OH group of donors, NAD or NADP as acceptor [GO:0016616]